{
  "gene": "UniProtKB:Q53FD0",
  "gene_symbol": "ZC2HC1C",
  "term_id": "UNKNOWN:0001",
  "term_label": "Unknown molecular function",
  "gene_name": "Zinc finger C2HC domain-containing protein 1C"
}